{
  "gene": "UniProtKB:Q8N139",
  "term_id": "GO:0042626",
  "gene_name": "ATP-binding cassette sub-family A member 6",
  "term_label": "ATPase-coupled transmembrane transporter activity",
  "gene_symbol": "ABCA6"
}